{
  "term_id": "UNKNOWN:0003",
  "gene_name": "Growth-regulated alpha protein",
  "gene_symbol": "CXCL1",
  "gene": "UniProtKB:P09341",
  "term_label": "Unknown cellular component"
}